heparanase activity [GO:0030305] (molecular function) Relationships: is a type of hydrolase activity, hydrolyzing O-glycosyl compounds [GO:0004553] Also known as: heparinase activity Definition: Catalysis of the cleavage of heparan sulfate; can degrade both heparan sulfate and heparin glycosaminoglycan chains. References: PMID:10916150